{
  "term_label": "Unknown cellular component",
  "term_id": "UNKNOWN:0003",
  "gene": "UniProtKB:Q8N386",
  "gene_name": "Leucine-rich repeat-containing protein 25",
  "gene_symbol": "LRRC25"
}